{
  "gene": "UniProtKB:P38405",
  "term_id": "GO:0031683",
  "gene_symbol": "GNAL",
  "gene_name": "Guanine nucleotide-binding protein G(olf) subunit alpha",
  "term_label": "G-protein beta/gamma-subunit complex binding"
}